{
  "gene": "UniProtKB:Q9HDB9",
  "gene_name": "Endogenous retrovirus group K member 5 Gag polyprotein",
  "gene_symbol": "ERVK-5",
  "term_label": "Unknown cellular component",
  "term_id": "UNKNOWN:0003"
}